{
  "term_id": "GO:0009897",
  "gene_symbol": "CD226",
  "term_label": "external side of plasma membrane",
  "gene": "UniProtKB:Q15762",
  "gene_name": "CD226 antigen"
}